{
  "gene_symbol": "DEFA6",
  "gene": "UniProtKB:Q01524",
  "term_id": "GO:0061844",
  "term_label": "antimicrobial humoral immune response mediated by antimicrobial peptide",
  "gene_name": "Defensin-6"
}